{
  "gene_name": "Chymotrypsinogen B2",
  "gene": "UniProtKB:Q6GPI1",
  "term_id": "GO:0006508",
  "term_label": "proteolysis",
  "gene_symbol": "CTRB2"
}